heme O catabolic process [GO:0048035] (biological process) Also known as: haem O catabolic process, haem O catabolism, heme O breakdown, heme O catabolism, heme O degradation Definition: The chemical reactions and pathways resulting in the breakdown of heme O, a derivative of heme containing a 17-carbon hydroxyethylfarnesyl side chain at position 8 of the tetrapyrrole macrocycle. Relationships: is_a heme catabolic process [GO:0042167] Sources: GOC:jid